Golgi to plasma membrane transport [GO:0006893] (biological process) Definition: The directed movement of substances from the Golgi to the plasma membrane in transport vesicles that move from the trans-Golgi network to the plasma membrane, where they fuse and release their contents by exocytosis. Also known as: Golgi to plasma membrane vesicle-mediated transport Subtypes: Golgi to plasma membrane protein transport [GO:0043001] Sources: ISBN:0716731363 Relationships: is a type of GO:0006892; is a type of vesicle-mediated transport to the plasma membrane [GO:0098876]